rostral hindbrain neuronal precursor cell proliferation [GO:0021931] (biological process) References: PMID:15157725 Sources: GOC:cls, GOC:dgh, GOC:dph, GOC:jid, GO_REF:0000021 Definition: The multiplication or reproduction of neuroblasts that will give rise to neurons of the lateral pontine nucleus and the locus ceruleus. Relationships: is a type of cell proliferation in external granule layer [GO:0021924]